{
  "gene_name": "Aquaporin-6",
  "term_label": "nitrate transmembrane transporter activity",
  "term_id": "GO:0015112",
  "gene_symbol": "AQP6",
  "gene": "UniProtKB:Q13520"
}